sensory perception of mechanical stimulus [GO:0050954] (biological process) Subtypes: GO:0007605, sensory perception of touch [GO:0050975], magnetoreception by sensory perception of mechanical stimulus [GO:0050979], sensory perception of wind [GO:0071063] Also known as: mechanosensory perception, perception of mechanical stimulus, chemi-mechanical coupling Sources: GOC:ai Definition: The series of events required for an organism to receive a sensory mechanical stimulus, convert it to a molecular signal, and recognize and characterize the signal. This is a neurological process. Relationships: is a type of GO:0007600